L-altrarate catabolic process [GO:1903663] (biological process) References: PMID:17649980 Sources: GOC:TermGenie, GO_REF:0000068 Definition: The chemical reactions and pathways resulting in the breakdown of L-altrarate. Also known as: L-altrarate(1-) breakdown, L-altrarate(1-) catabolism, L-altrarate(1-) degradation Relationships: is a type of carbohydrate catabolic process [GO:0016052]; is a type of aldaric acid catabolic process [GO:0019579]